{
  "gene_name": "Transmembrane protein 106B",
  "term_id": "GO:0007041",
  "gene": "UniProtKB:Q9NUM4",
  "gene_symbol": "TMEM106B",
  "term_label": "lysosomal transport"
}